RNA polymerase II intronic transcription regulatory region sequence-specific DNA binding [GO:0001162] (molecular function) Note: To minimize ambiguity in the use of the word "promoter" in GO, we have chosen the phrase "transcription regulatory region" to refer to all of the regulatory regions. Regulatory regions in the DNA which control initiation may include the "core promoter" where the basal transcription machinery binds, the "core promoter proximal region" where regulatory factors other than the basal machinery bind. There are also additional regulatory regions, in both the DNA and the RNA transcript, which regulate elongation or termination of transcription. Sources: GOC:txnOH Relationships: is a type of RNA polymerase II transcription regulatory region sequence-specific DNA binding [GO:0000977]; is a type of intronic transcription regulatory region sequence-specific DNA binding [GO:0001161] Definition: Binding to an RNA polymerase II intronic DNA sequence that regulates the transcription of the transcript it is contained within.